{
  "gene_name": "Vacuolar protein sorting-associated protein 37B",
  "gene": "UniProtKB:Q9H9H4",
  "term_label": "Unknown molecular function",
  "term_id": "UNKNOWN:0001",
  "gene_symbol": "VPS37B"
}